{
  "term_id": "GO:0008286",
  "gene_symbol": "PIK3R1",
  "gene": "UniProtKB:P27986",
  "term_label": "insulin receptor signaling pathway",
  "gene_name": "Phosphatidylinositol 3-kinase regulatory subunit alpha"
}